AMPylase activity [GO:0070733] (molecular function) Definition: Catalysis of the reaction: ATP + protein = diphosphate + adenylyl-protein; mediates the addition of an adenylyl (adenosine 5'-monophosphate; AMP group) to L-serine, L-threonine, and L-tyrosine residues in target proteins. Relationships: is a type of adenylyltransferase activity [GO:0070566] References: PMID:19039103, PMID:19362538, PMID:33947243 Sources: GOC:mah Also known as: adenosine monophosphate-protein transferase activity, AMPylator, protein adenylyltransferase activity